regulation of mammary stem cell proliferation [GO:2000101] (biological process) Sources: GOC:obol Relationships: is a type of regulation of cell population proliferation [GO:0042127]; regulates mammary stem cell proliferation [GO:0002174] Definition: Any process that modulates the frequency, rate or extent of mammary stem cell proliferation. Subtypes: negative regulation of mammary stem cell proliferation [GO:2000102], positive regulation of mammary stem cell proliferation [GO:2000103]